protein-RNA complex disassembly [GO:0032988] (biological process) Subtypes: spliceosomal complex disassembly [GO:0000390], GO:0035617 Also known as: RNA-protein complex disassembly, RNP complex disassembly, ribonucleoprotein complex disassembly Definition: The disaggregation of a protein-RNA complex into its constituent components. Relationships: is a type of protein-containing complex disassembly [GO:0032984]; is a type of protein-RNA complex organization [GO:0071826] Sources: GOC:mah